{
  "gene_name": "SET domain-containing protein 4",
  "term_label": "histone H3K4 methyltransferase activity",
  "gene": "UniProtKB:Q9NVD3",
  "term_id": "GO:0042800",
  "gene_symbol": "SETD4"
}